{
  "term_label": "extracellular space",
  "gene": "UniProtKB:Q9UBU2",
  "gene_symbol": "DKK2",
  "term_id": "GO:0005615",
  "gene_name": "Dickkopf-related protein 2"
}